{
  "term_id": "GO:0016020",
  "gene": "UniProtKB:Q96SU4",
  "term_label": "membrane",
  "gene_name": "Oxysterol-binding protein-related protein 9",
  "gene_symbol": "OSBPL9"
}